{
  "gene_name": "E3 ubiquitin-protein ligase MARCHF4",
  "gene": "UniProtKB:Q9P2E8",
  "term_id": "UNKNOWN:0002",
  "term_label": "Unknown biological process",
  "gene_symbol": "MARCHF4"
}